regulation of sterigmatocystin biosynthetic process [GO:0010913] (biological process) Subtypes: positive regulation of sterigmatocystin biosynthetic process [GO:0010914], GO:1900760 Definition: Any process that modulates the rate, frequency, or extent of sterigmatocystin biosynthesis. Sterigmatocystin biosynthetic processes are the chemical reactions and pathways resulting in the formation of sterigmatocystin, a carcinogenic mycotoxin produced in high yields by strains of the common molds. Relationships: is a type of regulation of secondary metabolite biosynthetic process [GO:1900376]; regulates sterigmatocystin biosynthetic process [GO:0045461] Sources: GOC:dph, GOC:tb